pulmonary valve morphogenesis [GO:0003184] (biological process) Definition: The process in which the structure of the pulmonary valve is generated and organized. Sources: GOC:mtg_heart Relationships: is a type of heart valve morphogenesis [GO:0003179]; is part of pulmonary valve development [GO:0003177]